{
  "term_label": "nervous system development",
  "gene_name": "Transcription factor AP-2-beta",
  "gene_symbol": "TFAP2B",
  "gene": "UniProtKB:Q92481",
  "term_id": "GO:0007399"
}